{
  "gene": "UniProtKB:O43323",
  "term_label": "cell fate specification",
  "gene_symbol": "DHH",
  "term_id": "GO:0001708",
  "gene_name": "Desert hedgehog protein"
}